regulation of phenazine biosynthetic process [GO:1900980] (biological process) Definition: Any process that modulates the frequency, rate or extent of phenazine biosynthetic process. Sources: GOC:TermGenie, GOC:mengo_curators Also known as: regulation of acridizine biosynthesis, regulation of acridizine biosynthetic process, regulation of azophenylene biosynthesis, regulation of azophenylene biosynthetic process, regulation of dibenzo-p-diazine biosynthesis, regulation of dibenzo-p-diazine biosynthetic process, regulation of dibenzopyrazine biosynthesis, regulation of dibenzopyrazine biosynthetic process Relationships: is a type of GO:0009889; regulates GO:0002047 Subtypes: GO:1900981, positive regulation of phenazine biosynthetic process [GO:1900982]